nuclear glucocorticoid receptor binding [GO:0035259] (molecular function) Relationships: is a type of nuclear receptor binding [GO:0016922] Subtypes: nuclear cortisol receptor binding [GO:0031961] Sources: GOC:bf Also known as: glucocorticoid receptor binding Definition: Binding to a nuclear glucocorticoid receptor.